{
  "gene_symbol": "MSH6",
  "term_label": "mismatched DNA binding",
  "term_id": "GO:0030983",
  "gene_name": "DNA mismatch repair protein Msh6",
  "gene": "UniProtKB:P52701"
}